glyceraldehyde-3-phosphate dehydrogenase [NAD(P)+] (phosphorylating) activity [GO:0043891] (MF) Relationships: is a type of oxidoreductase activity, acting on the aldehyde or oxo group of donors, NAD or NADP as acceptor [GO:0016620] Also known as: D-glyceraldehyde 3-phosphate:NAD(P)+ oxidoreductase (phosphorylating), glyceraldehyde-3-phosphate dehydrogenase (NAD(P)) (phosphorylating), triosephosphate dehydrogenase (NAD(P)), NAD(P)-dependent glyceraldehyde-3-phosphate dehydrogenase activity, triosephosphate dehydrogenase (NAD(P)+) Subtypes: glyceraldehyde-3-phosphate dehydrogenase (NAD+) (phosphorylating) activity [GO:0004365], GO:0047100 Definition: Catalysis of the reaction: D-glyceraldehyde 3-phosphate + phosphate + NAD(P)+ = 3-phospho-D-glyceroyl phosphate + NAD(P)H + H+. Sources: EC:1.2.1.59